{
  "term_id": "GO:2000048",
  "gene": "UniProtKB:Q5QGS0",
  "term_label": "negative regulation of cell-cell adhesion mediated by cadherin",
  "gene_name": "Neurite extension and migration factor",
  "gene_symbol": "NEXMIF"
}